magnetosome membrane [GO:0110146] (cellular component) Definition: The lipid bilayer surrounding a magnetosome. Relationships: is a type of GO:0031090; BFO_0000050 magnetosome [GO:0110143] References: PMID:27620945 Sources: GOC:aa